positive regulation of formation of radial glial scaffolds [GO:0061926] (biological process) Definition: Any process that increases the frequency, rate or extent of the formation of radial glial cell scaffolds. References: PMID:22076441 Also known as: positive regulation of radial glial scaffold formation, positive regulation of Bergmann fiber biosynthesis, positive regulation of Bergmann fiber formation Relationships: is a type of GO:0010770; is a type of GO:0061924; positively regulates GO:0021943